{
  "gene_symbol": "TGIF1",
  "term_label": "DNA-binding transcription repressor activity, RNA polymerase II-specific",
  "term_id": "GO:0001227",
  "gene_name": "Homeobox protein TGIF1",
  "gene": "UniProtKB:Q15583"
}